glutamate-1-semialdehyde 2,1-aminomutase activity [GO:0042286] (molecular function) Definition: Catalysis of the reaction: (S)-4-amino-5-oxopentanoate = 5-aminolevulinate. Sources: RHEA:14265 Also known as: (S)-4-amino-5-oxopentanoate 4,5-aminomutase activity, glutamate-1-semialdehyde aminotransferase activity Relationships: is a type of intramolecular aminotransferase activity [GO:0016869]